{
  "term_label": "detection of chemical stimulus involved in sensory perception of smell",
  "gene_symbol": "OR10J1",
  "gene": "UniProtKB:P30954",
  "gene_name": "Olfactory receptor 10J1",
  "term_id": "GO:0050911"
}